metanephric glomerular epithelial cell fate commitment [GO:0072315] (biological process) Definition: The process in which the developmental fate of a cell becomes restricted such that it will develop into a metanephric glomerular epithelial cell. Metanephric glomerular epithelial cells are specialized epithelial cells that form part of the metanephric glomerulus; there are two types, metanephric glomerular parietal epithelial cells and metanephric glomerular visceral epithelial cells. Subtypes: metanephric glomerular parietal epithelial cell fate commitment [GO:0072247], metanephric podocyte cell fate commitment [GO:0072250] Relationships: is a type of glomerular epithelial cell fate commitment [GO:0072314] Sources: GOC:mtg_kidney_jan10